{
  "gene_symbol": "RRP1B",
  "gene": "UniProtKB:Q14684",
  "term_id": "GO:0003713",
  "term_label": "transcription coactivator activity",
  "gene_name": "Ribosomal RNA processing protein 1 homolog B"
}